{
  "gene_name": "Immunoglobulin kappa constant",
  "term_label": "antigen binding",
  "gene_symbol": "IGKC",
  "gene": "UniProtKB:P01834",
  "term_id": "GO:0003823"
}